{
  "gene_name": "Archaemetzincin-2",
  "term_id": "UNKNOWN:0002",
  "term_label": "Unknown biological process",
  "gene_symbol": "AMZ2",
  "gene": "UniProtKB:Q86W34"
}